{
  "gene": "UniProtKB:P46663",
  "term_label": "G protein-coupled receptor signaling pathway",
  "gene_symbol": "BDKRB1",
  "term_id": "GO:0007186",
  "gene_name": "B1 bradykinin receptor"
}